{
  "gene_symbol": "GLRX",
  "term_id": "UNKNOWN:0003",
  "term_label": "Unknown cellular component",
  "gene_name": "Glutaredoxin-1",
  "gene": "UniProtKB:P35754"
}